{
  "gene_name": "Stomatin",
  "term_label": "Unknown biological process",
  "gene_symbol": "STOM",
  "term_id": "UNKNOWN:0002",
  "gene": "UniProtKB:P27105"
}